{
  "term_id": "GO:0032436",
  "gene_name": "PABIR family member 2",
  "gene": "UniProtKB:Q7Z309",
  "term_label": "positive regulation of proteasomal ubiquitin-dependent protein catabolic process",
  "gene_symbol": "PABIR2"
}